fungal-type cell wall (1->3)-beta-D-glucan metabolic process [GO:0071969] (biological process) Also known as: fungal-type cell wall 1,3-beta-D-glucan metabolic process, fungal-type cell wall 1,3-beta-glucan metabolism, fungal-type cell wall beta-1,3 glucan metabolic process, fungal-type cell wall beta-1,3 glucan metabolism Sources: GOC:mah Relationships: is a type of GO:0034407; is a type of fungal-type cell wall beta-glucan metabolic process [GO:0070879] Definition: The chemical reactions and pathways involving (1->3)-beta-D-glucans, compounds composed of glucose residues linked by (1->3)-beta-D-glucosidic bonds, found in the walls of fungi. Subtypes: ascospore wall (1->3)-beta-D-glucan metabolic process [GO:0034409], GO:0071970